{
  "gene_symbol": "APOB",
  "gene_name": "Apolipoprotein B-100",
  "gene": "UniProtKB:P04114",
  "term_label": "low-density lipoprotein particle receptor binding",
  "term_id": "GO:0050750"
}